{
  "term_label": "plasma membrane",
  "term_id": "GO:0005886",
  "gene_symbol": "NPTN",
  "gene_name": "Neuroplastin",
  "gene": "UniProtKB:Q9Y639"
}